nitric-oxide synthase inhibitor activity [GO:0036487] (molecular function) Relationships: is a type of GO:0004857; is_a nitric-oxide synthase regulator activity [GO:0030235]; negatively regulates GO:0004517 Also known as: NOS inhibitor activity, nitric oxide synthase inhibitor activity Definition: Binds to and stops, prevents or reduces the activity of nitric oxide synthase. References: PMID:17242280 Sources: GOC:BHF, GOC:rl